{
  "gene": "UniProtKB:Q676U5",
  "term_label": "phagophore assembly site membrane",
  "gene_name": "Autophagy-related protein 16-1",
  "term_id": "GO:0034045",
  "gene_symbol": "ATG16L1"
}